mini excitatory postsynaptic potential [GO:0098816] (biological process) Relationships: is a type of GO:0060079 Regulation: RO_0002211 by regulation of mini excitatory postsynaptic potential [GO:0061884]; positively regulated by positive regulation of mini excitatory postsynaptic potential [GO:0061885]; negatively regulated by GO:0061886 Sources: GOC:dos Definition: A process that leads to a temporary increase in postsynaptic potential due to the flow of positively charged ions into the postsynaptic cell, induced by the spontaneous release of a single vesicle of an excitatory neurotransmitter into the synapse.